{
  "term_label": "Unknown molecular function",
  "gene_symbol": "LETMD1",
  "term_id": "UNKNOWN:0001",
  "gene_name": "LETM1 domain-containing protein 1",
  "gene": "UniProtKB:Q6P1Q0"
}